{
  "term_id": "GO:0005886",
  "gene_symbol": "LYVE1",
  "term_label": "plasma membrane",
  "gene": "UniProtKB:Q9Y5Y7",
  "gene_name": "Lymphatic vessel endothelial hyaluronic acid receptor 1"
}